{
  "gene_symbol": "GABRG3",
  "gene_name": "Gamma-aminobutyric acid receptor subunit gamma-3",
  "gene": "UniProtKB:Q99928",
  "term_label": "GABA-A receptor complex",
  "term_id": "GO:1902711"
}